interleukin-18-mediated signaling pathway [GO:0035655] (biological process) Definition: The series of molecular signals initiated by interleukin-18 binding to its receptor on the surface of a target cell, and ending with the regulation of a downstream cellular process, e.g. transcription. Sources: GOC:BHF, GOC:bf, GOC:signaling Also known as: interleukin-18-mediated signalling pathway Relationships: is a type of GO:0019221; BFO_0000050 GO:0071351 Regulation: RO_0002211 by regulation of interleukin-18-mediated signaling pathway [GO:2000492]; negatively regulated by negative regulation of interleukin-18-mediated signaling pathway [GO:2000493]; positively regulated by positive regulation of interleukin-18-mediated signaling pathway [GO:2000494]